{
  "gene_name": "Taste receptor type 2 member 41",
  "gene_symbol": "TAS2R41",
  "term_id": "UNKNOWN:0001",
  "gene": "UniProtKB:P59536",
  "term_label": "Unknown molecular function"
}